{
  "term_label": "axonemal microtubule",
  "term_id": "GO:0005879",
  "gene_symbol": "EFHC1",
  "gene_name": "EF-hand domain-containing protein 1",
  "gene": "UniProtKB:Q5JVL4"
}